{
  "gene_symbol": "CRYBG1",
  "term_id": "UNKNOWN:0001",
  "term_label": "Unknown molecular function",
  "gene_name": "Beta_gamma crystallin domain-containing protein 1",
  "gene": "UniProtKB:Q9Y4K1"
}